{
  "term_label": "nucleolus",
  "gene_symbol": "RBM28",
  "gene": "UniProtKB:Q9NW13",
  "gene_name": "RNA-binding protein 28",
  "term_id": "GO:0005730"
}